{
  "gene_name": "Type 2 DNA topoisomerase 6 subunit B-like",
  "gene_symbol": "TOP6BL",
  "term_id": "GO:0007131",
  "gene": "UniProtKB:Q8N6T0",
  "term_label": "reciprocal meiotic recombination"
}